{
  "gene": "UniProtKB:P18433",
  "term_label": "signal transduction",
  "gene_symbol": "PTPRA",
  "gene_name": "Receptor-type tyrosine-protein phosphatase alpha",
  "term_id": "GO:0007165"
}